{
  "term_id": "GO:0005886",
  "gene_symbol": "NTRK1",
  "gene": "UniProtKB:P04629",
  "term_label": "plasma membrane",
  "gene_name": "High affinity nerve growth factor receptor"
}